{
  "term_id": "GO:0005829",
  "gene_name": "Autophagy-related protein 13",
  "gene_symbol": "ATG13",
  "gene": "UniProtKB:O75143",
  "term_label": "cytosol"
}